{
  "gene_name": "Small proline-rich protein 2E",
  "gene_symbol": "SPRR2E",
  "gene": "UniProtKB:P22531",
  "term_id": "GO:0030280",
  "term_label": "structural constituent of skin epidermis"
}